adult salivary gland morphogenesis [GO:0007437] (biological process) Sources: GOC:go_curators Definition: The process in which the anatomical structures of the adult salivary gland are generated and organized. Relationships: is a type of GO:0007435